{
  "gene_symbol": "BCL10",
  "term_id": "GO:0043422",
  "term_label": "protein kinase B binding",
  "gene_name": "B-cell lymphoma_leukemia 10",
  "gene": "UniProtKB:O95999"
}